{
  "gene": "UniProtKB:Q6ZSV7",
  "term_id": "UNKNOWN:0001",
  "term_label": "Unknown molecular function",
  "gene_name": "Putative uncharacterized protein FLJ45177",
  "gene_symbol": "Q6ZSV7"
}